poly(3-hydroxyalkanoate) metabolic process [GO:0042620] (biological process) References: PMID:9925580 Sources: GOC:jl Subtypes: poly(3-hydroxyalkanoate) biosynthetic process [GO:0042621] Also known as: PHA metabolic process, PHA metabolism, poly(3-hydroxyalkanoate) metabolism Definition: The chemical reactions and pathways involving poly(3-hydroxyalkanoates), polyesters of 3-hydroxyacids produced as intracellular granules by a large variety of bacteria. Relationships: is_a metabolic process [GO:0008152]